{
  "term_id": "GO:0042361",
  "gene_name": "Cytochrome P450 4F2",
  "term_label": "menaquinone catabolic process",
  "gene": "UniProtKB:P78329",
  "gene_symbol": "CYP4F2"
}